negative regulation of germinal center formation [GO:0002635] (biological process) Relationships: is a type of regulation of germinal center formation [GO:0002634]; is a type of GO:0002823; is a type of GO:0051093; negatively regulates germinal center formation [GO:0002467] Definition: Any process that stops, prevents, or reduces the frequency, rate, or extent of germinal center formation. Also known as: down regulation of germinal center formation, down-regulation of germinal center formation, downregulation of germinal center formation, inhibition of germinal center formation Sources: GOC:add